{
  "term_id": "UNKNOWN:0001",
  "gene_name": "Inactive N-acetyllactosaminide alpha-1,3-galactosyltransferase",
  "gene": "UniProtKB:Q4G0N0",
  "term_label": "Unknown molecular function",
  "gene_symbol": "GGTA1"
}